{
  "term_label": "cytosol",
  "gene_symbol": "FAM72D",
  "term_id": "GO:0005829",
  "gene": "UniProtKB:Q6L9T8",
  "gene_name": "Protein FAM72D"
}